{
  "gene_symbol": "OSBPL11",
  "term_label": "Unknown biological process",
  "gene_name": "Oxysterol-binding protein-related protein 11",
  "term_id": "UNKNOWN:0002",
  "gene": "UniProtKB:Q9BXB4"
}